{
  "gene": "UniProtKB:Q86YV0",
  "term_id": "GO:0005096",
  "gene_name": "RAS protein activator like-3",
  "term_label": "GTPase activator activity",
  "gene_symbol": "RASAL3"
}